{
  "gene_name": "Solute carrier family 23 member 3",
  "gene": "UniProtKB:Q6PIS1",
  "term_id": "UNKNOWN:0002",
  "term_label": "Unknown biological process",
  "gene_symbol": "SLC23A3"
}